{
  "gene_symbol": "RPA3",
  "term_label": "DNA replication factor A complex",
  "term_id": "GO:0005662",
  "gene": "UniProtKB:P35244",
  "gene_name": "Replication protein A 14 kDa subunit"
}